{
  "gene_symbol": "ARPC5",
  "gene_name": "Actin-related protein 2_3 complex subunit 5",
  "term_label": "Arp2/3 protein complex",
  "gene": "UniProtKB:O15511",
  "term_id": "GO:0005885"
}